{
  "gene_name": "Laminin subunit beta-2",
  "gene_symbol": "LAMB2",
  "term_label": "substrate adhesion-dependent cell spreading",
  "term_id": "GO:0034446",
  "gene": "UniProtKB:P55268"
}